{
  "gene_symbol": "SPOCK1",
  "term_label": "extracellular space",
  "gene_name": "Testican-1",
  "gene": "UniProtKB:Q08629",
  "term_id": "GO:0005615"
}